{
  "term_id": "GO:0001937",
  "gene": "UniProtKB:O75829",
  "term_label": "negative regulation of endothelial cell proliferation",
  "gene_name": "Leukocyte cell-derived chemotaxin 1",
  "gene_symbol": "CNMD"
}